{
  "gene_symbol": "LYSET",
  "gene_name": "Lysosomal enzyme trafficking factor",
  "term_id": "UNKNOWN:0003",
  "term_label": "Unknown cellular component",
  "gene": "UniProtKB:Q8N6I4"
}